{
  "gene_symbol": "RPS25",
  "gene_name": "Small ribosomal subunit protein eS25",
  "gene": "UniProtKB:P62851",
  "term_label": "cytosolic small ribosomal subunit",
  "term_id": "GO:0022627"
}